{
  "term_label": "Unknown molecular function",
  "gene_symbol": "EME1",
  "gene_name": "Crossover junction endonuclease EME1",
  "gene": "UniProtKB:Q96AY2",
  "term_id": "UNKNOWN:0001"
}